{
  "gene_name": "Interferon regulatory factor 3",
  "term_id": "GO:0000978",
  "gene": "UniProtKB:Q14653",
  "gene_symbol": "IRF3",
  "term_label": "RNA polymerase II cis-regulatory region sequence-specific DNA binding"
}